positive regulation of endothelial cell migration [GO:0010595] (biological process) Definition: Any process that increases the rate, frequency, or extent of the orderly movement of an endothelial cell into the extracellular matrix to form an endothelium. Relationships: is a type of regulation of endothelial cell migration [GO:0010594]; is a type of positive regulation of cell migration [GO:0030335]; positively regulates endothelial cell migration [GO:0043542] Sources: GOC:BHF, GOC:dph, GOC:tb Subtypes: GO:0043536, positive regulation of endothelial cell chemotaxis [GO:2001028]